apical recycling endosome [GO:0090653] (cellular component) Relationships: is a type of recycling endosome [GO:0055037]; is part of apical cytoplasm [GO:0090651] Definition: Tubulo-vesicular structure located in the apical cytoplasm that participates in apical cargo recycling in polarized epithelial cells. References: PMID:12669082, PMID:16394106, PMID:17494872, PMID:21170358, PMID:9405315